negative regulation of cellotriose transport [GO:1900286] (BP) Definition: Any process that stops, prevents or reduces the frequency, rate or extent of cellotriose transport. Also known as: down regulation of cellotriose transport, down-regulation of cellotriose transport, downregulation of cellotriose transport, inhibition of cellotriose transport Relationships: is a type of negative regulation of transport [GO:0051051]; is a type of regulation of cellotriose transport [GO:1900285]; negatively regulates GO:2001096 Sources: GOC:TermGenie, GOC:mengo_curators